{
  "gene_name": "Synaptotagmin-3",
  "term_label": "SNARE binding",
  "gene_symbol": "SYT3",
  "gene": "UniProtKB:Q9BQG1",
  "term_id": "GO:0000149"
}